symbiont-mediated stabilization of host tight cell-cell junction [GO:0098864] (biological process) References: PMID:25838979 Also known as: modification by symbiont of host tight cell-cell junction, stabilization of host tight cell-cell junction Definition: The process in which a symbiont organism that stabilizes the its host tight cell-cell junctions, making them less dynamic. The tight junction is a cell-cell junction that seals cells together in an epithelium in a way that prevents even small molecules from leaking from one side of the sheet to the other, and plays a role in the inflammatory response of the host. Relationships: is a type of symbiont-mediated perturbation of host tight cell-cell junction [GO:0098865]